{
  "term_id": "GO:0000981",
  "term_label": "DNA-binding transcription factor activity, RNA polymerase II-specific",
  "gene_name": "Cytoplasmic polyadenylated homeobox-like protein",
  "gene": "UniProtKB:A0A1W2PPM1",
  "gene_symbol": "CPHXL"
}